{
  "term_id": "GO:0005509",
  "gene": "UniProtKB:P06703",
  "term_label": "calcium ion binding",
  "gene_name": "Protein S100-A6",
  "gene_symbol": "S100A6"
}